{
  "gene_symbol": "PROC",
  "term_label": "proteolysis",
  "term_id": "GO:0006508",
  "gene_name": "Vitamin K-dependent protein C",
  "gene": "UniProtKB:P04070"
}